{
  "gene_symbol": "IGHJ3",
  "term_label": "Unknown biological process",
  "gene_name": "Immunoglobulin heavy joining 3 (Fragment)",
  "term_id": "UNKNOWN:0002",
  "gene": "UniProtKB:A0A0J9YW14"
}